{
  "gene": "UniProtKB:Q496F6",
  "gene_name": "CMRF35-like molecule 2",
  "term_id": "GO:0007165",
  "term_label": "signal transduction",
  "gene_symbol": "CD300E"
}